oxidoreductase activity, acting on a heme group of donors, nitrogenous group as acceptor [GO:0016677] (molecular function) Subtypes: GO:0050140 Definition: Catalysis of an oxidation-reduction (redox) reaction in which a heme group acts as a hydrogen or electron donor and reduces a nitrogenous group. Also known as: oxidoreductase activity, acting on haem group of donors, nitrogenous group as acceptor Relationships: is a type of oxidoreductase activity, acting on a heme group of donors [GO:0016675] Sources: GOC:jl